methane biosynthetic process from dimethylamine [GO:2001129] (biological process) Relationships: is a type of GO:0009308; is a type of methanogenesis [GO:0015948] Definition: The chemical reactions and pathways resulting in the formation of a methane from a dimethylamine. Regulation: regulated by regulation of methane biosynthetic process from dimethylamine [GO:1900318]; negatively regulated by negative regulation of methane biosynthetic process from dimethylamine [GO:1900319]; RO_0002213 by GO:1900320 Sources: GOC:mengo_curators